bacterial pre-replicative complex [GO:0036389] (cellular component) Relationships: is_a pre-replicative complex [GO:0036387]; has part DnaA-oriC complex [GO:1990101] Definition: A protein-DNA complex that forms at the bacterial oriC during the initial step of DNA replication and allows the origin to become competent, or 'licensed', for replication. Also known as: bacterial pre-RC References: PMID:19833870, PMID:21035377 Sources: GOC:bf, GOC:bhm, GOC:jh2, Wikipedia:Pre-replication_complex